{
  "gene_symbol": "ZSCAN20",
  "gene_name": "Zinc finger and SCAN domain-containing protein 20",
  "gene": "UniProtKB:P17040",
  "term_label": "RNA polymerase II cis-regulatory region sequence-specific DNA binding",
  "term_id": "GO:0000978"
}